{
  "gene_name": "Zinc finger protein 30",
  "term_id": "GO:0005634",
  "gene_symbol": "ZNF30",
  "gene": "UniProtKB:P17039",
  "term_label": "nucleus"
}